calcium activated galactosylceramide scrambling [GO:0061591] (biological process) References: PMID:23532839 Sources: GOC:krc Definition: The movement of a population of galactosylceramide molecules from one leaflet of the plasma membrane bilayer to the opposite leaflet as a result of a calcium stimulus. Relationships: is a type of calcium activated phospholipid scrambling [GO:0061588]